{
  "gene_name": "Double-stranded RNA-specific adenosine deaminase",
  "gene": "UniProtKB:P55265",
  "gene_symbol": "ADAR",
  "term_id": "GO:0008251",
  "term_label": "tRNA-specific adenosine deaminase activity"
}